killing by virus of host cell by post-segregational killing [GO:0044696] (biological process) Note: Note that this process occurs after the cell division partitioning event. Relationships: is a type of GO:0001907 Also known as: killing by virus of host cell by PSK, killing by virus of host cell by toxin-antitoxin system References: PMID:11222604 Sources: GOC:bf, GOC:jl, Wikipedia:Toxin-antitoxin_system Definition: The process by which a virus causes the death of daughter cells which do not contain its genes after host cell division, by a mechanism of post-segregational killing (PSK). The extrachromosomal viral DNA consist of two genes; the product of the second is long lived and toxic, while the product of the first is short lived and antagonizes the lethal action of the toxin. Daughter cells that do not contain the viral extrachromosomal element are killed by the long lived toxin, while daughter cells that do contain the viral extrachromosomal element are protected by the action of the short lived antitoxin it encodes.